{
  "gene_symbol": "H2AB1",
  "gene_name": "Histone H2A-Bbd type 1",
  "term_id": "GO:0030527",
  "term_label": "structural constituent of chromatin",
  "gene": "UniProtKB:P0C5Y9"
}